{
  "gene": "UniProtKB:Q9HAR2",
  "gene_symbol": "ADGRL3",
  "term_label": "plasma membrane",
  "term_id": "GO:0005886",
  "gene_name": "Adhesion G protein-coupled receptor L3"
}